{
  "term_label": "Unknown molecular function",
  "gene": "UniProtKB:Q9C005",
  "gene_symbol": "DPY30",
  "term_id": "UNKNOWN:0001",
  "gene_name": "Protein dpy-30 homolog"
}